{
  "gene_name": "Keratin, type II cytoskeletal 1",
  "term_id": "GO:0031424",
  "term_label": "keratinization",
  "gene": "UniProtKB:P04264",
  "gene_symbol": "KRT1"
}